glycoside-pentoside-hexuronide:cation symporter activity [GO:0015486] (molecular function) Subtypes: GO:0015488 Definition: Enables the transfer of a solute or solutes from one side of a membrane to the other according to the reaction: (glycoside, pentoside or hexuronide)(out) + monovalent cation(out) = (glycoside, pentoside or hexuronide)(in) + monovalent cation(in). The cation is Na+, Li+ or H+. Relationships: is a type of carbohydrate:monoatomic cation symporter activity [GO:0005402] Sources: TC:2.A.2.-.-